{
  "gene_name": "DBH-like monooxygenase protein 1",
  "gene": "UniProtKB:Q6UVY6",
  "gene_symbol": "MOXD1",
  "term_id": "GO:0005507",
  "term_label": "copper ion binding"
}